cellular response to tacrolimus [GO:0072748] (biological process) Definition: Any process that results in a change in state or activity of a cell (in terms of movement, secretion, enzyme production, gene expression, etc.) as a result of a tacrolimus (FK506) stimulus. Sources: GOC:mah Also known as: cellular response to FK506, cellular response to tacrolimus hydrate Relationships: is a type of response to tacrolimus [GO:1901327]; is_a cellular response to nitrogen compound [GO:1901699]; is_a cellular response to oxygen-containing compound [GO:1901701]